{
  "gene": "UniProtKB:P33076",
  "term_label": "positive regulation of MHC class I biosynthetic process",
  "term_id": "GO:0045345",
  "gene_name": "MHC class II transactivator",
  "gene_symbol": "CIITA"
}